{
  "term_id": "GO:0072542",
  "gene_name": "Serine_threonine-protein phosphatase 4 regulatory subunit 3A",
  "gene_symbol": "PPP4R3A",
  "term_label": "protein phosphatase activator activity",
  "gene": "UniProtKB:Q6IN85"
}